poly(ADP-ribose) glycohydrolase activity [GO:0004649] (molecular function) Relationships: is a type of hydrolase activity, hydrolyzing O-glycosyl compounds [GO:0004553] Definition: Catalysis of the hydrolysis of poly(ADP-ribose) at glycosidic (1''-2') linkage of ribose-ribose bond to produce free ADP-ribose. Sources: EC:3.2.1.143